{
  "gene": "UniProtKB:Q12905",
  "term_label": "double-stranded RNA binding",
  "term_id": "GO:0003725",
  "gene_name": "Interleukin enhancer-binding factor 2",
  "gene_symbol": "ILF2"
}